{
  "gene_name": "Putative nucleotidyltransferase MAB21L1",
  "gene_symbol": "MAB21L1",
  "term_label": "Unknown molecular function",
  "gene": "UniProtKB:Q13394",
  "term_id": "UNKNOWN:0001"
}